{
  "gene": "UniProtKB:Q96EF6",
  "term_label": "SCF ubiquitin ligase complex",
  "gene_symbol": "FBXO17",
  "gene_name": "F-box only protein 17",
  "term_id": "GO:0019005"
}